{
  "term_label": "histone binding",
  "gene": "UniProtKB:Q99733",
  "term_id": "GO:0042393",
  "gene_name": "Nucleosome assembly protein 1-like 4",
  "gene_symbol": "NAP1L4"
}